{
  "term_label": "Unknown biological process",
  "gene_name": "Ornithine decarboxylase antizyme 3",
  "term_id": "UNKNOWN:0002",
  "gene": "UniProtKB:Q9UMX2",
  "gene_symbol": "OAZ3"
}